{
  "term_id": "GO:0005634",
  "term_label": "nucleus",
  "gene": "UniProtKB:O00110",
  "gene_name": "Putative transcription factor ovo-like protein 3",
  "gene_symbol": "OVOL3"
}